apical part of cell [GO:0045177] (cellular component) Relationships: is a type of cellular anatomical structure [GO:0110165] Also known as: apical region of cell Definition: The region of a polarized cell that forms a tip or is distal to a base. For example, in a polarized epithelial cell, the apical region has an exposed surface and lies opposite to the basal lamina that separates the epithelium from other tissue. Sources: GOC:mah, ISBN:0815316194